{
  "gene_name": "Trefoil factor 2",
  "term_label": "extracellular space",
  "gene": "UniProtKB:Q03403",
  "gene_symbol": "TFF2",
  "term_id": "GO:0005615"
}